{
  "gene": "UniProtKB:Q9NPC8",
  "gene_name": "Homeobox protein SIX2",
  "term_id": "GO:0000981",
  "gene_symbol": "SIX2",
  "term_label": "DNA-binding transcription factor activity, RNA polymerase II-specific"
}